{
  "term_label": "clathrin-coated pit",
  "gene_symbol": "FCHO1",
  "gene": "UniProtKB:O14526",
  "term_id": "GO:0005905",
  "gene_name": "F-BAR domain only protein 1"
}